{
  "term_label": "extracellular space",
  "gene": "UniProtKB:P55107",
  "gene_symbol": "GDF10",
  "gene_name": "Growth_differentiation factor 10",
  "term_id": "GO:0005615"
}